{
  "gene": "UniProtKB:Q9Y257",
  "term_id": "GO:0005886",
  "gene_symbol": "KCNK6",
  "gene_name": "Potassium channel subfamily K member 6",
  "term_label": "plasma membrane"
}